{
  "term_label": "Unknown biological process",
  "gene": "UniProtKB:O14981",
  "gene_symbol": "BTAF1",
  "term_id": "UNKNOWN:0002",
  "gene_name": "TATA-binding protein-associated factor 172"
}